{
  "gene_symbol": "SLC2A12",
  "gene": "UniProtKB:Q8TD20",
  "term_id": "GO:0072359",
  "gene_name": "Solute carrier family 2, facilitated glucose transporter member 12",
  "term_label": "circulatory system development"
}